positive regulation of neutrophil mediated cytotoxicity [GO:0070960] (biological process) Relationships: is a type of GO:0001912; is a type of positive regulation of myeloid leukocyte mediated immunity [GO:0002888]; is a type of regulation of neutrophil mediated cytotoxicity [GO:0070948]; positively regulates GO:0070942 Also known as: positive regulation of neutrophil mediated cell killing, up regulation of neutrophil mediated cytotoxicity, up-regulation of neutrophil mediated cytotoxicity, upregulation of neutrophil mediated cytotoxicity, activation of neutrophil mediated cytotoxicity, stimulation of neutrophil mediated cytotoxicity Sources: GOC:add, GOC:mah Subtypes: positive regulation of neutrophil mediated killing of symbiont cell [GO:0070961] Definition: Any process that increases the frequency, rate or extent of the directed killing of a target cell by a neutrophil.